{
  "gene": "UniProtKB:Q8NGA8",
  "gene_name": "Olfactory receptor 4F17",
  "term_id": "UNKNOWN:0002",
  "gene_symbol": "OR4F17",
  "term_label": "Unknown biological process"
}